chondroitin sulfate proteoglycan metabolic process [GO:0050654] (biological process) Also known as: chondroitin sulfate proteoglycan metabolism, chondroitin sulphate proteoglycan metabolic process, chondroitin sulphate proteoglycan metabolism Subtypes: chondroitin sulfate proteoglycan catabolic process [GO:0030207], chondroitin sulfate proteoglycan biosynthetic process [GO:0050650] Relationships: is a type of proteoglycan metabolic process [GO:0006029] References: PMID:17239763 Definition: The chemical reactions and pathways involving chondroitin sulfate proteoglycans, which consist of a core protein linked to a chondroitin sulfate glycosaminoglycan. The chondroitin sulfate chain is composed of the repeating disaccharide unit beta-(1,4)-D-glucuronic acid-beta-(1,3)-N-acetyl-D-galactosamine, the latter of which can be O-sulfated.